{
  "gene_symbol": "SMPD2",
  "term_id": "GO:0005901",
  "gene_name": "Sphingomyelin phosphodiesterase 2",
  "term_label": "caveola",
  "gene": "UniProtKB:O60906"
}